{
  "gene": "UniProtKB:Q9UJJ7",
  "term_label": "pseudouridine synthase activity",
  "gene_name": "RNA pseudouridylate synthase domain-containing protein 1",
  "term_id": "GO:0009982",
  "gene_symbol": "RPUSD1"
}